{
  "gene_symbol": "OR5AC2",
  "term_label": "odorant binding",
  "gene_name": "Olfactory receptor 5AC2",
  "gene": "UniProtKB:Q9NZP5",
  "term_id": "GO:0005549"
}